{
  "term_label": "protein phosphatase binding",
  "gene": "UniProtKB:Q13615",
  "term_id": "GO:0019903",
  "gene_symbol": "MTMR3",
  "gene_name": "Myotubularin-related protein 3"
}